{
  "gene": "UniProtKB:P60468",
  "term_id": "GO:0016020",
  "term_label": "membrane",
  "gene_symbol": "SEC61B",
  "gene_name": "Protein transport protein Sec61 subunit beta"
}